{
  "gene_symbol": "AK5",
  "term_id": "GO:0005829",
  "gene": "UniProtKB:Q9Y6K8",
  "gene_name": "Adenylate kinase isoenzyme 5",
  "term_label": "cytosol"
}